{
  "gene_symbol": "MAGEA11",
  "term_id": "GO:0000122",
  "gene_name": "Melanoma-associated antigen 11",
  "term_label": "negative regulation of transcription by RNA polymerase II",
  "gene": "UniProtKB:P43364"
}